positive regulation of lipid transport across blood-brain barrier [GO:1903002] (biological process) Definition: Any process that activates or increases the frequency, rate or extent of lipid transport across blood-brain barrier. References: PMID:24345162 Sources: GOC:TermGenie, GOC:sjp, GO_REF:0000058 Also known as: positive regulation of lipid transport across blood brain barrier, up regulation of lipid transport across blood brain barrier, up-regulation of lipid transport across blood brain barrier, upregulation of lipid transport across blood brain barrier, activation of lipid transport across blood brain barrier Relationships: is a type of positive regulation of lipid transport [GO:0032370]; is a type of positive regulation of transport across blood-brain barrier [GO:0150201]; is a type of regulation of lipid transport across blood-brain barrier [GO:1903000]; positively regulates lipid transport across blood-brain barrier [GO:1990379]